inner membrane pellicle complex [GO:0070258] (cellular component) References: PMID:12456714 Sources: GOC:mah Definition: A membrane structure formed of two closely aligned lipid bilayers that lie beneath the plasma membrane and form part of the pellicle surrounding an apicomplexan parasite cell. Relationships: is_a GO:0110165; is part of pellicle [GO:0020039] Also known as: inner membrane complex